{
  "term_label": "regulation of mitotic nuclear division",
  "term_id": "GO:0007088",
  "gene_symbol": "CUL7",
  "gene": "UniProtKB:Q14999",
  "gene_name": "Cullin-7"
}